{
  "term_label": "regulation of transcription by RNA polymerase II",
  "gene": "UniProtKB:Q8WYA1",
  "gene_name": "Basic helix-loop-helix ARNT-like protein 2",
  "gene_symbol": "BMAL2",
  "term_id": "GO:0006357"
}